{
  "term_label": "nucleus",
  "gene_symbol": "HSPB7",
  "gene": "UniProtKB:Q9UBY9",
  "gene_name": "Heat shock protein beta-7",
  "term_id": "GO:0005634"
}